{
  "gene_symbol": "RNF216P1",
  "term_label": "Unknown biological process",
  "gene": "UniProtKB:Q6NUR6",
  "term_id": "UNKNOWN:0002",
  "gene_name": "Putative protein RNF216-like"
}